{
  "gene_name": "Apolipoprotein C-II",
  "term_label": "low-density lipoprotein particle",
  "gene": "UniProtKB:P02655",
  "term_id": "GO:0034362",
  "gene_symbol": "APOC2"
}